regulation of post-embryonic root development [GO:2000069] (biological process) Definition: Any process that modulates the frequency, rate or extent of post-embryonic root development. Subtypes: regulation of lateral root development [GO:2000023] Relationships: is a type of GO:0048580; is a type of regulation of root development [GO:2000280]; regulates post-embryonic root development [GO:0048528] Sources: GOC:obol